{
  "gene_symbol": "LGALS9C",
  "term_id": "GO:0032689",
  "gene": "UniProtKB:Q6DKI2",
  "gene_name": "Galectin-9C",
  "term_label": "negative regulation of type II interferon production"
}